{
  "gene_symbol": "GSKIP",
  "gene_name": "GSK3B-interacting protein",
  "gene": "UniProtKB:Q9P0R6",
  "term_label": "regulation of Wnt signaling pathway",
  "term_id": "GO:0030111"
}